{
  "gene_name": "G antigen 12I",
  "term_label": "Unknown cellular component",
  "gene": "UniProtKB:P0CL82",
  "gene_symbol": "GAGE12I",
  "term_id": "UNKNOWN:0003"
}